{
  "gene_name": "Fibrillin-3",
  "gene_symbol": "FBN3",
  "gene": "UniProtKB:Q75N90",
  "term_label": "extracellular matrix structural constituent",
  "term_id": "GO:0005201"
}